{
  "gene_symbol": "TRIM45",
  "gene": "UniProtKB:Q9H8W5",
  "term_id": "UNKNOWN:0002",
  "term_label": "Unknown biological process",
  "gene_name": "E3 ubiquitin-protein ligase TRIM45"
}